glycol biosynthetic process [GO:0042845] (biological process) Subtypes: butanediol biosynthetic process [GO:0034079], phthiocerol biosynthetic process [GO:0097040] Definition: The chemical reactions and pathways resulting in the formation of glycol, a diol in which the two hydroxy groups are on different carbon atoms, usually but not necessarily adjacent. Also known as: dihydric alcohol biosynthesis, dihydric alcohol biosynthetic process, glycol anabolism, glycol biosynthesis, glycol formation, glycol synthesis Relationships: is a type of GO:0034312; is a type of GO:0042844 Sources: GOC:curators